homocysteine metabolic process [GO:0050667] (BP) Also known as: Hcy metabolic process, Hcy metabolism, homocysteine metabolism Definition: The chemical reactions and pathways involving homocysteine, the amino acid alpha-amino-gamma-mercaptobutanoic acid. Homocysteine is an important intermediate in the metabolic reactions of its S-methyl derivative, methionine. Sources: ISBN:0198506732 Relationships: is a type of GO:0000096; is a type of non-proteinogenic amino acid metabolic process [GO:0170041]; is a type of alpha-amino acid metabolic process [GO:1901605] Subtypes: transsulfuration [GO:0019346], homocysteine catabolic process [GO:0043418], homocysteine biosynthetic process [GO:0071268]